database_cross_reference [oboInOwl#hasDbXref]